{
  "gene": "UniProtKB:Q8WYJ6",
  "term_label": "synaptic vesicle",
  "gene_symbol": "SEPTIN1",
  "gene_name": "Septin-1",
  "term_id": "GO:0008021"
}